{
  "term_label": "extracellular space",
  "term_id": "GO:0005615",
  "gene_name": "Myeloperoxidase",
  "gene": "UniProtKB:P05164",
  "gene_symbol": "MPO"
}